{
  "term_label": "precatalytic spliceosome",
  "term_id": "GO:0071011",
  "gene": "UniProtKB:A8MWD9",
  "gene_name": "Putative small nuclear ribonucleoprotein G-like protein 15",
  "gene_symbol": "SNRPGP15"
}